{
  "gene_name": "Putative RNA-binding protein Luc7-like 2",
  "term_label": "U1 snRNP",
  "gene_symbol": "LUC7L2",
  "gene": "UniProtKB:Q9Y383",
  "term_id": "GO:0005685"
}